positive regulation of glucocorticoid secretion [GO:2000851] (biological process) Definition: Any process that activates or increases the frequency, rate or extent of glucocorticoid secretion. Sources: GOC:sl Relationships: is a type of positive regulation of corticosteroid hormone secretion [GO:2000848]; is a type of regulation of glucocorticoid secretion [GO:2000849]; positively regulates glucocorticoid secretion [GO:0035933] Subtypes: positive regulation of cortisol secretion [GO:0051464], positive regulation of corticosterone secretion [GO:2000854]